{
  "term_id": "GO:0005634",
  "gene": "UniProtKB:P48742",
  "term_label": "nucleus",
  "gene_name": "LIM_homeobox protein Lhx1",
  "gene_symbol": "LHX1"
}